biotin catabolic process [GO:0042367] (biological process) Also known as: biotin breakdown, biotin catabolism, biotin degradation, vitamin B7 catabolic process, vitamin B7 catabolism, vitamin H catabolic process, vitamin H catabolism Definition: The chemical reactions and pathways resulting in the breakdown of biotin, cis-tetrahydro-2-oxothieno(3,4-d)imidazoline-4-valeric acid. Sources: ISBN:0198506732 Relationships: is a type of biotin metabolic process [GO:0006768]; is a type of water-soluble vitamin catabolic process [GO:0042365]; is a type of amide catabolic process [GO:0043605]; is a type of sulfur compound catabolic process [GO:0044273]; is a type of monocarboxylic acid catabolic process [GO:0072329]